endoplasmic reticulum N-glycan trimming [GO:0140277] (biological process) Definition: The trimming, in the ER, of the protein newly attached N-glycan by glucosidases and mannosidases to produce high mannose-type N-glycans. Relationships: is a type of N-glycan processing [GO:0006491] Also known as: ER N-glycan trimming References: PMID:30858582